{
  "gene_symbol": "REEP3",
  "gene": "UniProtKB:Q6NUK4",
  "term_id": "GO:0005881",
  "gene_name": "Receptor expression-enhancing protein 3",
  "term_label": "cytoplasmic microtubule"
}